positive regulation of cellular response to transforming growth factor beta stimulus [GO:1903846] (biological process) References: PMID:22269326 Sources: GOC:BHF, GOC:BHF_miRNA, GOC:TermGenie, GOC:rph, GO_REF:0000058 Relationships: is a type of positive regulation of response to stimulus [GO:0048584]; is_a GO:1903844; RO_0002213 GO:0071560 Subtypes: positive regulation of transforming growth factor beta receptor signaling pathway [GO:0030511] Definition: Any process that activates or increases the frequency, rate or extent of cellular response to transforming growth factor beta stimulus. Also known as: positive regulation of cellular response to TGF-beta stimulus, positive regulation of cellular response to TGFbeta stimulus, up regulation of cellular response to TGF-beta stimulus, up regulation of cellular response to TGFbeta stimulus, up regulation of cellular response to transforming growth factor beta stimulus, up-regulation of cellular response to TGF-beta stimulus, up-regulation of cellular response to TGFbeta stimulus, up-regulation of cellular response to transforming growth factor beta stimulus, upregulation of cellular response to TGF-beta stimulus, upregulation of cellular response to TGFbeta stimulus, upregulation of cellular response to transforming growth factor beta stimulus, activation of cellular response to TGF-beta stimulus, activation of cellular response to TGFbeta stimulus, activation of cellular response to transforming growth factor beta stimulus